negative regulation of sensory perception of sweet taste [GO:1904657] (biological process) References: PMID:1716172 Sources: GOC:TermGenie, GOC:mr, GO_REF:0000058 Also known as: down regulation of sensory perception of sweet taste, down regulation of sweet taste perception, down-regulation of sensory perception of sweet taste, down-regulation of sweet taste perception, downregulation of sensory perception of sweet taste, downregulation of sweet taste perception, negative regulation of sweet taste perception, inhibition of sensory perception of sweet taste, inhibition of sweet taste perception Definition: Any process that stops, prevents or reduces the frequency, rate or extent of sensory perception of sweet taste. Relationships: is_a negative regulation of nervous system process [GO:0031645]; is_a regulation of sensory perception of sweet taste [GO:1904656]; negatively regulates sensory perception of sweet taste [GO:0050916]